{
  "gene_symbol": "FMOD",
  "term_id": "UNKNOWN:0001",
  "gene": "UniProtKB:Q06828",
  "term_label": "Unknown molecular function",
  "gene_name": "Fibromodulin"
}